5,10-methylenetetrahydrofolate-dependent methyltransferase activity [GO:0042083] (molecular function) Subtypes: thymidylate synthase activity [GO:0004799], thymidylate synthase (FAD) activity [GO:0050797] Relationships: is a type of methyltransferase activity [GO:0008168] Definition: Catalysis of the transfer of a methyl group to an acceptor molecule; dependent on the presence of 5,10-methylenetetrahydrofolate. Sources: GOC:ai